{
  "term_id": "GO:0000224",
  "gene": "UniProtKB:Q96IV0",
  "gene_symbol": "NGLY1",
  "gene_name": "Peptide-N(4)-(N-acetyl-beta-glucosaminyl)asparagine amidase",
  "term_label": "peptide-N4-(N-acetyl-beta-glucosaminyl)asparagine amidase activity"
}